{
  "gene_name": "Actin-related protein 2_3 complex subunit 5-like protein",
  "term_label": "cortical cytoskeleton",
  "gene_symbol": "ARPC5L",
  "gene": "UniProtKB:Q9BPX5",
  "term_id": "GO:0030863"
}